{
  "gene_name": "Histatin-1",
  "term_id": "GO:0061844",
  "gene_symbol": "HTN1",
  "term_label": "antimicrobial humoral immune response mediated by antimicrobial peptide",
  "gene": "UniProtKB:P15515"
}